meiotic mismatch repair involved in reciprocal meiotic recombination [GO:0010777] (biological process) Definition: A system for the identification and correction of base-base mismatches, small insertion-deletion loops, and regions of heterology that are present in duplex DNA formed with strands from two recombining molecules resulting in meiotic recombination. Meiotic recombination is the cell cycle process in which double strand breaks are formed and repaired through a double Holliday junction intermediate. Sources: GOC:dph, GOC:tb Relationships: is a type of meiotic mismatch repair [GO:0000710]; BFO_0000050 reciprocal meiotic recombination [GO:0007131]